His-Purkinje system cell differentiation [GO:0060932] (biological process) Definition: The process in which a relatively unspecialized cell acquires the specialized structural and/or functional features of a cell of the His-Purkinje system. These cells form the fibers regulate cardiac muscle contraction in the ventricles. Subtypes: atrioventricular bundle cell differentiation [GO:0003167], Purkinje myocyte differentiation [GO:0003168] Relationships: is a type of GO:0055007; is part of His-Purkinje system development [GO:0003164] Sources: GOC:mtg_heart